folate:monoatomic anion antiporter activity [GO:0008518] (molecular function) Also known as: folate:anion antiporter activity, reduced folate carrier activity, reduced folate transmembrane transporter activity, reduced folate transporter Relationships: is a type of monoatomic anion transmembrane transporter activity [GO:0008509]; is a type of folic acid transmembrane transporter activity [GO:0008517]; is a type of antiporter activity [GO:0015297] References: PMID:21568705, PMID:24745983 Sources: GOC:mtg_transport, TC:2.A.48 Definition: Enables the transfer of a solute or solutes from one side of a membrane to the other according to the reaction: Folate derivative (out) + anion (in) = folate derivative (in) + anion (out). The Reduced Folate Carrier (RCF(SLC19A1) acts by an antiport mechanism. RCF carries several folate derivatives: MTX, PMX, ratitrexed, pralatrexate, 5-methyl THF, and 5-formyl THF.